negative regulation of sprouting of injured axon [GO:0048688] (BP) Also known as: down regulation of sprouting of injured axon, down-regulation of sprouting of injured axon, downregulation of sprouting of injured axon, inhibition of sprouting of injured axon Sources: GOC:dgh, GOC:dph, GOC:jid, GOC:lm Definition: Any process that stops, prevents, or reduces the frequency, rate or extent of sprouting of an injured axon. Subtypes: GO:0048692, GO:0048695, GO:1905943 Relationships: is a type of GO:0030308; is a type of negative regulation of developmental growth [GO:0048640]; is a type of negative regulation of axon regeneration [GO:0048681]; is_a regulation of sprouting of injured axon [GO:0048686]; negatively regulates sprouting of injured axon [GO:0048682]